{
  "gene_symbol": "ZNF723",
  "term_label": "RNA polymerase II cis-regulatory region sequence-specific DNA binding",
  "gene": "UniProtKB:P0DPD5",
  "term_id": "GO:0000978",
  "gene_name": "Zinc finger protein 723"
}